{
  "gene_name": "Chromosome alignment-maintaining phosphoprotein 1",
  "gene_symbol": "CHAMP1",
  "term_id": "GO:0034501",
  "term_label": "protein localization to kinetochore",
  "gene": "UniProtKB:Q96JM3"
}